{
  "gene_name": "High affinity copper uptake protein 1",
  "gene": "UniProtKB:O15431",
  "term_id": "GO:0015677",
  "gene_symbol": "SLC31A1",
  "term_label": "copper ion import"
}